{
  "gene": "UniProtKB:Q9HCJ2",
  "gene_symbol": "LRRC4C",
  "gene_name": "Leucine-rich repeat-containing protein 4C",
  "term_id": "GO:0005886",
  "term_label": "plasma membrane"
}